{
  "gene": "UniProtKB:A0A075B6K5",
  "term_label": "immune response",
  "gene_symbol": "IGLV3-9",
  "gene_name": "Immunoglobulin lambda variable 3-9",
  "term_id": "GO:0006955"
}